{
  "gene": "UniProtKB:Q7RTW8",
  "term_label": "Unknown molecular function",
  "gene_name": "Otoancorin",
  "gene_symbol": "OTOA",
  "term_id": "UNKNOWN:0001"
}